{
  "gene_symbol": "PSEN1",
  "term_label": "Notch signaling pathway",
  "term_id": "GO:0007219",
  "gene_name": "Presenilin-1",
  "gene": "UniProtKB:P49768"
}